{
  "gene_symbol": "JAML",
  "gene": "UniProtKB:Q86YT9",
  "term_label": "neutrophil chemotaxis",
  "gene_name": "Junctional adhesion molecule-like",
  "term_id": "GO:0030593"
}